{
  "gene": "UniProtKB:Q8WTV0",
  "gene_name": "Scavenger receptor class B member 1",
  "term_label": "lipid binding",
  "term_id": "GO:0008289",
  "gene_symbol": "SCARB1"
}